{
  "gene_symbol": "GSK3A",
  "term_id": "GO:0032436",
  "term_label": "positive regulation of proteasomal ubiquitin-dependent protein catabolic process",
  "gene": "UniProtKB:P49840",
  "gene_name": "Glycogen synthase kinase-3 alpha"
}